calcium:sodium antiporter activity [GO:0005432] (molecular function) Definition: Enables the transfer of a solute or solutes from one side of a membrane to the other according to the reaction: Ca2+(in) + Na+(out) = Ca2+(out) + Na+(in). References: PMID:16371597 Sources: GOC:curators Also known as: sodium/calcium exchanger, mitochondrial sodium/calcium ion exchange, sodium:calcium exchange Subtypes: calcium, potassium:sodium antiporter activity [GO:0008273], calcium:sodium antiporter activity involved in regulation of cardiac muscle cell membrane potential [GO:0086038] Relationships: is a type of sodium ion transmembrane transporter activity [GO:0015081]; is a type of calcium:monoatomic cation antiporter activity [GO:0015368]